polytene chromosome puff [GO:0005703] (cellular component) Definition: A swelling at a site along the length of a polytene chromosome, thought to be the site of active transcription. Relationships: is a type of chromosomal region [GO:0098687]; is part of GO:0005700 Sources: GOC:bf, ISBN:0120649012